{
  "gene_name": "Probable E3 ubiquitin-protein ligase MID2",
  "gene_symbol": "MID2",
  "term_id": "GO:0005874",
  "term_label": "microtubule",
  "gene": "UniProtKB:Q9UJV3"
}